iron-nicotianamine transmembrane transporter activity [GO:0051980] (molecular function) Relationships: is a type of iron chelate transmembrane transporter activity [GO:0015603] Definition: Enables the transfer of the iron chelate iron-nicotianamine (Fe-NA) from one side of a membrane to the other. Also known as: Fe-NA chelate transporter activity References: PMID:20625001 Sources: GOC:ai